{
  "gene_symbol": "OR6F1",
  "gene_name": "Olfactory receptor 6F1",
  "term_id": "GO:0004984",
  "term_label": "olfactory receptor activity",
  "gene": "UniProtKB:Q8NGZ6"
}